{
  "term_label": "Unknown molecular function",
  "gene": "UniProtKB:Q9HAD4",
  "gene_symbol": "WDR41",
  "term_id": "UNKNOWN:0001",
  "gene_name": "WD repeat-containing protein 41"
}